{
  "gene": "UniProtKB:Q13351",
  "gene_symbol": "KLF1",
  "term_label": "nucleus",
  "gene_name": "Krueppel-like factor 1",
  "term_id": "GO:0005634"
}